CD70 receptor binding [GO:0042614] (molecular function) Definition: Binding to a CD70, a receptor found on the surface of most activated B cells and some activated T cells. Relationships: is a type of signaling receptor binding [GO:0005102] Also known as: CD27L binding, CD27 receptor activity Sources: GOC:jl, ISBN:0120781859